mRNA catabolic process [GO:0006402] (BP) Also known as: mRNA breakdown, mRNA catabolism, mRNA degradation, mRNA decay Relationships: is a type of RNA catabolic process [GO:0006401]; is a type of negative regulation of gene expression [GO:0010629]; is a type of mRNA metabolic process [GO:0016071] Subtypes: nuclear-transcribed mRNA catabolic process [GO:0000956], mitochondrial mRNA catabolic process [GO:0000958], polyadenylation-dependent mRNA catabolic process [GO:0071047], GO:0141065, polyuridylation-dependent mRNA catabolic process [GO:1990074] Definition: The chemical reactions and pathways resulting in the breakdown of mRNA, messenger RNA, which is responsible for carrying the coded genetic 'message', transcribed from DNA, to sites of protein assembly at the ribosomes. Sources: ISBN:0198506732 Regulation: regulated by regulation of mRNA catabolic process [GO:0061013]; positively regulated by positive regulation of mRNA catabolic process [GO:0061014]; RO_0002212 by negative regulation of mRNA catabolic process [GO:1902373]